{
  "term_label": "Unknown molecular function",
  "term_id": "UNKNOWN:0001",
  "gene_symbol": "CCDC144A",
  "gene": "UniProtKB:A2RUR9",
  "gene_name": "Coiled-coil domain-containing protein 144A"
}